phosphatidylinositol-5-phosphate binding [GO:0010314] (molecular function) Sources: GOC:bf, GOC:tair_curators Definition: Binding to phosphatidylinositol-5-phosphate, a derivative of phosphatidylinositol in which the inositol ring is phosphorylated at the 5' position. Relationships: is a type of phosphatidylinositol phosphate binding [GO:1901981]